piperine biosynthetic process [GO:0160181] (biological process) Definition: The chemical reactions and pathways resulting in the formation of piperine. References: PMID:33435446, PMID:33833371 Relationships: is a type of alkaloid biosynthetic process [GO:0009821]; is_a GO:0043604